positive regulation of enamel mineralization [GO:0070175] (biological process) Definition: Any process that activates or increases the frequency, rate or extent of enamel mineralization, the deposition of calcium salts in tooth enamel. Relationships: is a type of positive regulation of tooth mineralization [GO:0070172]; is a type of GO:0070173; positively regulates enamel mineralization [GO:0070166] Sources: GOC:BHF, GOC:mah